{
  "term_id": "GO:0005096",
  "gene": "UniProtKB:Q9Y3L3",
  "term_label": "GTPase activator activity",
  "gene_symbol": "SH3BP1",
  "gene_name": "SH3 domain-binding protein 1"
}